{
  "gene_symbol": "THEMIS",
  "gene": "UniProtKB:Q8N1K5",
  "gene_name": "Protein THEMIS",
  "term_label": "cytoplasm",
  "term_id": "GO:0005737"
}